{
  "gene_name": "Pepsin A-5",
  "gene_symbol": "PGA5",
  "term_label": "aspartic-type endopeptidase activity",
  "term_id": "GO:0004190",
  "gene": "UniProtKB:P0DJD9"
}